{
  "term_id": "UNKNOWN:0002",
  "gene": "UniProtKB:Q14201",
  "gene_symbol": "BTG3",
  "term_label": "Unknown biological process",
  "gene_name": "Protein BTG3"
}